{
  "term_label": "DNA-binding transcription factor activity, RNA polymerase II-specific",
  "gene_symbol": "FOXL3",
  "gene": "UniProtKB:A0A1W2PRP0",
  "gene_name": "Forkhead box protein L3",
  "term_id": "GO:0000981"
}